{
  "term_id": "GO:0005737",
  "gene_name": "Serine_threonine-protein kinase pim-1",
  "gene": "UniProtKB:P11309",
  "gene_symbol": "PIM1",
  "term_label": "cytoplasm"
}